{
  "term_id": "GO:0000724",
  "gene": "UniProtKB:O94761",
  "gene_name": "ATP-dependent DNA helicase Q4",
  "term_label": "double-strand break repair via homologous recombination",
  "gene_symbol": "RECQL4"
}